{
  "gene_symbol": "ADAM15",
  "gene_name": "Disintegrin and metalloproteinase domain-containing protein 15",
  "term_id": "GO:0007229",
  "term_label": "integrin-mediated signaling pathway",
  "gene": "UniProtKB:Q13444"
}